{
  "gene": "UniProtKB:O95069",
  "term_id": "GO:0022841",
  "gene_name": "Potassium channel subfamily K member 2",
  "gene_symbol": "KCNK2",
  "term_label": "potassium ion leak channel activity"
}